{
  "gene_name": "Cilia- and flagella-associated protein 410",
  "gene": "UniProtKB:O43822",
  "gene_symbol": "CFAP410",
  "term_id": "GO:0007010",
  "term_label": "cytoskeleton organization"
}